{
  "gene_name": "E3 ubiquitin-protein ligase RNF114",
  "gene_symbol": "RNF114",
  "gene": "UniProtKB:Q9Y508",
  "term_label": "Unknown cellular component",
  "term_id": "UNKNOWN:0003"
}